glucosidase II complex [GO:0017177] (cellular component) Also known as: alpha-glucosidase II complex Relationships: is_a GO:0140534; is a type of glucosidase complex [GO:1902687] Note: Note that alpha-glucosidase I functions as a monomer, and therefore does not have a corresponding cellular component term. References: PMID:10464333, PMID:8910335 Definition: A heterodimeric complex that catalyzes the trimming of glucose residues from N-linked core glycans on newly synthesized glycoproteins.